{
  "gene": "UniProtKB:P48730",
  "gene_name": "Casein kinase I isoform delta",
  "term_id": "GO:0005737",
  "gene_symbol": "CSNK1D",
  "term_label": "cytoplasm"
}